plastid acetate CoA-transferase complex [GO:0032283] (cellular component) Definition: An acetate CoA-transferase complex located in the stroma of a plastid. Sources: GOC:mah Relationships: is a type of acetate CoA-transferase complex [GO:0009329]; is part of plastid acetyl-CoA carboxylase complex [GO:0032282]